cellular response to haloperidol [GO:1905120] (biological process) Note: Note that this term is in the subset of terms that should not be used for direct manual annotation of gene products. It was created to be used for cross-referencing by other ontologies. Direct annotations to this term may be amended during annotation QC. Definition: Any process that results in a change in state or activity of a cell (in terms of movement, secretion, enzyme production, gene expression, etc.) as a result of a haloperidol stimulus. Relationships: is a type of cellular response to alcohol [GO:0097306]; is a type of cellular response to ketone [GO:1901655]; is a type of GO:1901699; is a type of response to haloperidol [GO:1905119] References: PMID:24751813 Sources: GOC:TermGenie, GOC:dw, GO_REF:0000071